{
  "term_id": "GO:0035267",
  "gene": "UniProtKB:Q9Y230",
  "gene_symbol": "RUVBL2",
  "term_label": "NuA4 histone acetyltransferase complex",
  "gene_name": "RuvB-like 2"
}